{
  "gene_name": "Fragile X messenger ribonucleoprotein 1",
  "gene": "UniProtKB:Q06787",
  "gene_symbol": "FMR1",
  "term_label": "positive regulation of long-term neuronal synaptic plasticity",
  "term_id": "GO:0048170"
}